{
  "gene": "UniProtKB:P20248",
  "term_label": "microtubule organizing center",
  "term_id": "GO:0005815",
  "gene_symbol": "CCNA2",
  "gene_name": "Cyclin-A2"
}